extrinsic component of postsynaptic endocytic zone [GO:0098893] (cellular component) Sources: GOC:autophagy, GOC:mf Definition: The component of the postsynaptic endocytic zone membrane consisting of gene products and protein complexes that are loosely bound to one of its surfaces, but not integrated into the hydrophobic region. Relationships: is_a extrinsic component of postsynaptic membrane [GO:0098890]; is part of postsynaptic endocytic zone membrane [GO:0098844]